{
  "gene_name": "Extracellular sulfatase Sulf-2",
  "term_id": "GO:0009986",
  "gene": "UniProtKB:Q8IWU5",
  "term_label": "cell surface",
  "gene_symbol": "SULF2"
}